GTPase regulator activity [GO:0030695] (molecular function) Definition: Binds to and modulates the activity of a GTPase. Also known as: small GTPase regulator activity, small GTPase regulatory/interacting protein activity Sources: GOC:mah Relationships: is a type of nucleoside-triphosphatase regulator activity [GO:0060589]; RO_0002211 GTPase activity [GO:0003924] Subtypes: guanyl-nucleotide exchange factor activity [GO:0005085], guanyl-nucleotide exchange factor adaptor activity [GO:0005091], GDP-dissociation inhibitor activity [GO:0005092], GO:0005095, GTPase activator activity [GO:0005096]